{
  "gene": "UniProtKB:P08519",
  "term_label": "Unknown molecular function",
  "term_id": "UNKNOWN:0001",
  "gene_symbol": "LPA",
  "gene_name": "Apolipoprotein(a)"
}